{
  "gene_symbol": "CD200R1L",
  "gene_name": "Cell surface glycoprotein CD200 receptor 2",
  "gene": "UniProtKB:Q6Q8B3",
  "term_id": "GO:0009897",
  "term_label": "external side of plasma membrane"
}